{
  "term_id": "GO:0005737",
  "gene_symbol": "CAMKV",
  "gene_name": "CaM kinase-like vesicle-associated protein",
  "term_label": "cytoplasm",
  "gene": "UniProtKB:Q8NCB2"
}